{
  "gene": "UniProtKB:P0C7X4",
  "term_label": "ferric iron binding",
  "gene_name": "Putative ferritin heavy polypeptide-like 19",
  "gene_symbol": "FTH1P19",
  "term_id": "GO:0008199"
}